{
  "gene_symbol": "PPP1R37",
  "term_id": "UNKNOWN:0002",
  "term_label": "Unknown biological process",
  "gene": "UniProtKB:O75864",
  "gene_name": "Protein phosphatase 1 regulatory subunit 37"
}